{
  "gene_symbol": "CFAP300",
  "term_id": "UNKNOWN:0003",
  "gene": "UniProtKB:Q9BRQ4",
  "gene_name": "Cilia- and flagella-associated protein 300",
  "term_label": "Unknown cellular component"
}